{
  "gene_symbol": "CYP27C1",
  "term_label": "retinoic acid binding",
  "gene_name": "Cytochrome P450 27C1",
  "gene": "UniProtKB:Q4G0S4",
  "term_id": "GO:0001972"
}